{
  "term_id": "GO:0008284",
  "gene_symbol": "IL6R",
  "gene": "UniProtKB:P08887",
  "term_label": "positive regulation of cell population proliferation",
  "gene_name": "Interleukin-6 receptor subunit alpha"
}